{
  "gene": "UniProtKB:P17022",
  "gene_name": "Zinc finger protein 18",
  "gene_symbol": "ZNF18",
  "term_label": "regulation of transcription by RNA polymerase II",
  "term_id": "GO:0006357"
}